{
  "gene": "UniProtKB:Q9UIA9",
  "gene_name": "Exportin-7",
  "term_label": "nuclear pore",
  "gene_symbol": "XPO7",
  "term_id": "GO:0005643"
}